{
  "gene_name": "Zinc finger protein 549",
  "gene_symbol": "ZNF549",
  "term_id": "GO:0005634",
  "term_label": "nucleus",
  "gene": "UniProtKB:Q6P9A3"
}